alpha-(1->3)-fucosyltransferase activity [GO:0046920] (molecular function) Subtypes: 4-galactosyl-N-acetylglucosaminide 3-alpha-L-fucosyltransferase activity [GO:0017083], glycoprotein 3-alpha-L-fucosyltransferase activity [GO:0018392] Definition: Catalysis of the transfer of an L-fucosyl group from GDP-beta-L-fucose to an acceptor molecule to form an alpha-(1->3) linkage. Also known as: alpha(1,3)-fucosyltransferase activity, alpha-(1,3)-fucosyltransferase activity, alpha-1,3-fucosyltransferase activity Sources: GOC:ai Relationships: is a type of fucosyltransferase activity [GO:0008417]